{
  "gene_symbol": "ZDHHC1",
  "term_id": "GO:0019706",
  "term_label": "protein-cysteine S-palmitoyltransferase activity",
  "gene_name": "Palmitoyltransferase ZDHHC1",
  "gene": "UniProtKB:Q8WTX9"
}